{
  "term_label": "neuron projection",
  "gene": "UniProtKB:P16157",
  "term_id": "GO:0043005",
  "gene_name": "Ankyrin-1",
  "gene_symbol": "ANK1"
}